{
  "gene_name": "Hemoglobin subunit alpha",
  "gene": "UniProtKB:P69905",
  "term_label": "erythrocyte development",
  "gene_symbol": "HBA2",
  "term_id": "GO:0048821"
}